positive regulation of phosphatidylinositol biosynthetic process [GO:0010513] (biological process) Subtypes: GO:1902648 Definition: Any process that increases the frequency, rate or extent of the chemical reactions and pathways resulting in the formation of phosphatidylinositol. Sources: GOC:dph, GOC:tb, GOC:vw Relationships: is a type of GO:0010511; is a type of GO:0071073; positively regulates phosphatidylinositol biosynthetic process [GO:0006661]